carbamate kinase activity [GO:0008804] (molecular function) Definition: Catalysis of the reaction: ATP + NH3 + CO2 = ADP + carbamoyl phosphate. Sources: EC:2.7.2.2 Also known as: ATP:carbamate phosphotransferase activity, CKase activity, carbamoyl phosphokinase activity, carbamyl phosphokinase activity Relationships: is_a kinase activity [GO:0016301]; is a type of phosphotransferase activity, carboxyl group as acceptor [GO:0016774]